{
  "term_id": "GO:0003924",
  "term_label": "GTPase activity",
  "gene_name": "Ras-related protein Rab-3A",
  "gene": "UniProtKB:P20336",
  "gene_symbol": "RAB3A"
}